{
  "term_label": "basolateral plasma membrane",
  "gene_symbol": "SCRIB",
  "term_id": "GO:0016323",
  "gene": "UniProtKB:Q14160",
  "gene_name": "Protein scribble homolog"
}